{
  "gene_name": "Kelch repeat and BTB domain-containing protein 2",
  "term_id": "GO:0005737",
  "term_label": "cytoplasm",
  "gene_symbol": "KBTBD2",
  "gene": "UniProtKB:Q8IY47"
}